FMN biosynthetic process [GO:0009398] (biological process) Definition: The chemical reactions and pathways resulting in the formation of FMN, the oxidized form of flavin mononucleotide (riboflavin 5'-(dihydrogen phosphate)), which acts as a coenzyme for a number of oxidative enzymes including NADH dehydrogenase. Relationships: is a type of ribonucleoside monophosphate biosynthetic process [GO:0009156]; is a type of ribonucleotide biosynthetic process [GO:0009260]; is a type of flavin-containing compound biosynthetic process [GO:0042727]; is a type of FMN metabolic process [GO:0046444] Sources: GOC:ai Also known as: FMN anabolism, FMN biosynthesis, FMN formation, FMN synthesis